{
  "gene_name": "Large ribosomal subunit protein eL15",
  "gene_symbol": "RPL15",
  "term_label": "cytosolic large ribosomal subunit",
  "term_id": "GO:0022625",
  "gene": "UniProtKB:P61313"
}